{
  "gene": "UniProtKB:Q9BV47",
  "gene_symbol": "DUSP26",
  "gene_name": "Dual specificity protein phosphatase 26",
  "term_label": "protein tyrosine/serine/threonine phosphatase activity",
  "term_id": "GO:0008138"
}